arachidonate 12(S)-lipoxygenase activity [GO:0004052] (molecular function) Also known as: leukotriene A4 synthase, 12-lipoxygenase activity, 12Delta-lipoxygenase activity, 12S-lipoxygenase activity, C-12 lipoxygenase activity, LTA4 synthase activity, arachidonate:oxygen 12-oxidoreductase activity, delta12-lipoxygenase activity Sources: EC:1.13.11.31, RHEA:10428 Relationships: is a type of oxidoreductase activity, acting on single donors with incorporation of molecular oxygen, incorporation of two atoms of oxygen [GO:0016702] Definition: Catalysis of the reaction: arachidonate + O2 = (5Z,8Z,10E,12S,14Z)-12-hydroperoxyicosa-5,8,10,14-tetraenoate.